cellular detoxification of acetone [GO:0140977] (biological process) References: PMID:22314896, PMID:26958851 Definition: Any process carried out at the cellular level that reduces or removes the toxicity of acetone. These may include chemical modification, for example to methylglyoxal. Relationships: is_a cellular detoxification [GO:1990748]